regulation of intracellular protein transport [GO:0033157] (biological process) Relationships: is a type of regulation of intracellular transport [GO:0032386]; is a type of GO:0051223; regulates intracellular protein transport [GO:0006886] Sources: GOC:mah Subtypes: GO:0042306, GO:0046825, regulation of protein exit from endoplasmic reticulum [GO:0070861], positive regulation of intracellular protein transport [GO:0090316], negative regulation of intracellular protein transport [GO:0090317], regulation of post-translational protein targeting to membrane, translocation [GO:0120235], regulation of protein targeting to vacuolar membrane [GO:1900483], regulation of protein targeting to vacuole involved in autophagy [GO:1904051], regulation of axo-dendritic protein transport [GO:1905126], regulation of endosome to plasma membrane protein transport [GO:1905749], regulation of protein localization by the Cvt pathway [GO:2001159] Definition: Any process that modulates the frequency, rate or extent of the directed movement of proteins within cells.